{
  "gene_name": "Nuclear autoantigenic sperm protein",
  "term_label": "CENP-A containing chromatin assembly",
  "gene": "UniProtKB:P49321",
  "term_id": "GO:0034080",
  "gene_symbol": "NASP"
}